{
  "gene": "UniProtKB:Q14739",
  "term_label": "cholesterol biosynthetic process",
  "gene_name": "Delta(14)-sterol reductase LBR",
  "term_id": "GO:0006695",
  "gene_symbol": "LBR"
}